{
  "gene_symbol": "TBC1D2B",
  "term_id": "GO:0005096",
  "gene_name": "TBC1 domain family member 2B",
  "term_label": "GTPase activator activity",
  "gene": "UniProtKB:Q9UPU7"
}